integrase activity [GO:0008907] (molecular function) Subtypes: site-specific recombinase activity [GO:0009009], retroviral integrase activity [GO:0044823] Sources: GOC:mah Definition: Catalysis of the integration of one DNA segment into another. Relationships: is a type of catalytic activity, acting on DNA [GO:0140097]; is part of GO:0015074